{
  "gene": "UniProtKB:Q5M775",
  "gene_name": "Cytospin-B",
  "gene_symbol": "SPECC1",
  "term_label": "microtubule organizing center",
  "term_id": "GO:0005815"
}